{
  "gene_symbol": "MPP1",
  "term_label": "plasma membrane",
  "gene_name": "55 kDa erythrocyte membrane protein",
  "gene": "UniProtKB:Q00013",
  "term_id": "GO:0005886"
}